{
  "gene_name": "WD repeat-containing protein 82",
  "gene_symbol": "WDR82",
  "gene": "UniProtKB:Q6UXN9",
  "term_label": "Unknown biological process",
  "term_id": "UNKNOWN:0002"
}